{
  "term_id": "GO:0016020",
  "term_label": "membrane",
  "gene_name": "Uncharacterized protein C20orf173",
  "gene": "UniProtKB:Q96LM9",
  "gene_symbol": "C20orf173"
}